{
  "term_label": "nucleus",
  "gene_name": "Pancreas_duodenum homeobox protein 1",
  "gene": "UniProtKB:P52945",
  "term_id": "GO:0005634",
  "gene_symbol": "PDX1"
}